{
  "gene": "UniProtKB:Q6ZWT7",
  "gene_name": "Lysophospholipid acyltransferase 2",
  "gene_symbol": "MBOAT2",
  "term_id": "GO:0036152",
  "term_label": "phosphatidylethanolamine acyl-chain remodeling"
}